{
  "term_id": "GO:0008233",
  "term_label": "peptidase activity",
  "gene": "UniProtKB:Q8NDH3",
  "gene_name": "Probable aminopeptidase NPEPL1",
  "gene_symbol": "NPEPL1"
}